collagen V binding [GO:0070052] (molecular function) Relationships: is a type of collagen binding [GO:0005518] Definition: Binding to a type V collagen trimer. Sources: GOC:BHF, GOC:mah